carbon dioxide binding [GO:1902670] (molecular function) Relationships: is a type of GO:0036094 References: PMID:15491402 Sources: GOC:TermGenie, GOC:bhm, GO_REF:0000067 Definition: Binding to carbon dioxide. Also known as: CO2 binding